{
  "term_id": "GO:0010754",
  "gene_symbol": "PDE11A",
  "gene": "UniProtKB:Q9HCR9",
  "term_label": "negative regulation of receptor guanylyl cyclase signaling pathway",
  "gene_name": "Dual 3',5'-cyclic-AMP and -GMP phosphodiesterase 11A"
}